{
  "term_label": "regulation of RNA splicing",
  "gene_name": "Zinc finger CCCH domain-containing protein 10",
  "gene": "UniProtKB:Q96K80",
  "gene_symbol": "ZC3H10",
  "term_id": "GO:0043484"
}